carotenoid dioxygenase activity [GO:0010436] (molecular function) Definition: Catalysis of the oxidative cleavage of carotenoids. References: PMID:16459333 Also known as: carotenoid-cleaving dioxygenase Relationships: is a type of GO:0016702 Subtypes: 9,10 (9', 10')-carotenoid-cleaving dioxygenase activity [GO:0010437], GO:0045549, carotenoid isomerooxygenase activity [GO:0106422]